{
  "gene": "UniProtKB:Q13609",
  "term_label": "deoxyribonuclease I activity",
  "term_id": "GO:0004530",
  "gene_name": "Deoxyribonuclease gamma",
  "gene_symbol": "DNASE1L3"
}